{
  "gene": "UniProtKB:P26367",
  "gene_name": "Paired box protein Pax-6",
  "term_label": "type B pancreatic cell differentiation",
  "term_id": "GO:0003309",
  "gene_symbol": "PAX6"
}